{
  "gene_symbol": "ESRP2",
  "gene": "UniProtKB:Q9H6T0",
  "term_label": "mRNA binding",
  "term_id": "GO:0003729",
  "gene_name": "Epithelial splicing regulatory protein 2"
}